T=169 icosahedral viral capsid [GO:0039628] (cellular component) Sources: GOC:plm, VZ:10117 Also known as: T=169 icosahedral capsid Definition: The protein coat that surrounds the infective nucleic acid in some virus particles where the subunits (capsomeres) are arranged to form an icosahedron with T=169 symmetry. T=169 icosahedral capsid is composed of 12 pentameric and 1680 hexameric capsomeres for a total of 10140 capsid proteins. Relationships: is a type of icosahedral viral capsid [GO:0019030]